{
  "term_label": "vesicle-mediated transport",
  "gene_symbol": "ARL6",
  "term_id": "GO:0016192",
  "gene": "UniProtKB:Q9H0F7",
  "gene_name": "ADP-ribosylation factor-like protein 6"
}